{
  "gene_symbol": "HNRNPDL",
  "gene_name": "Heterogeneous nuclear ribonucleoprotein D-like",
  "term_label": "nucleoplasm",
  "term_id": "GO:0005654",
  "gene": "UniProtKB:O14979"
}